{
  "gene_name": "Epoxide hydrolase 4",
  "term_label": "hydrolase activity",
  "term_id": "GO:0016787",
  "gene": "UniProtKB:Q8IUS5",
  "gene_symbol": "EPHX4"
}